negative regulation of mesoderm formation [GO:1905903] (biological process) Relationships: is a type of GO:1905902; is a type of negative regulation of mesoderm development [GO:2000381]; negatively regulates mesoderm formation [GO:0001707] Also known as: down regulation of mesoderm formation, down-regulation of mesoderm formation, downregulation of mesoderm formation, inhibition of mesoderm formation References: PMID:23939491 Sources: GOC:BHF, GOC:BHF_miRNA, GOC:TermGenie, GOC:rph, GO_REF:0000058 Definition: Any process that stops, prevents or reduces the frequency, rate or extent of mesoderm formation.